phloem or xylem histogenesis [GO:0010087] (biological process) Relationships: is a type of GO:0009888 Subtypes: GO:0010088, xylem development [GO:0010089] Definition: The process whose specific outcome is the progression of phloem and/or xylem over time, from formation to the mature structure. An example of this process is found in Arabidopsis thaliana. Sources: GOC:mtg_sensu, GOC:tb Also known as: vascular tissue development, vascular tissue histogenesis